{
  "term_id": "GO:0005044",
  "term_label": "scavenger receptor activity",
  "gene": "UniProtKB:Q8WTV0",
  "gene_symbol": "SCARB1",
  "gene_name": "Scavenger receptor class B member 1"
}